{
  "gene_symbol": "HBG1",
  "gene": "UniProtKB:P69891",
  "term_id": "GO:0005833",
  "term_label": "hemoglobin complex",
  "gene_name": "Hemoglobin subunit gamma-1"
}